{
  "term_id": "GO:0005886",
  "term_label": "plasma membrane",
  "gene_symbol": "PCDHB16",
  "gene_name": "Protocadherin beta-16",
  "gene": "UniProtKB:Q9NRJ7"
}